{
  "term_id": "GO:0000226",
  "term_label": "microtubule cytoskeleton organization",
  "gene_symbol": "TOGARAM2",
  "gene_name": "TOG array regulator of axonemal microtubules protein 2",
  "gene": "UniProtKB:Q6ZUX3"
}